strigolactone biosynthetic process [GO:1901601] (biological process) Sources: GOC:TermGenie Definition: The chemical reactions and pathways resulting in the formation of strigolactone. Relationships: is a type of sesquiterpenoid biosynthetic process [GO:0016106]; is a type of lactone biosynthetic process [GO:1901336]; is_a strigolactone metabolic process [GO:1901600] Also known as: strigolactone anabolism, strigolactone biosynthesis, strigolactone formation, strigolactone synthesis